{
  "gene_symbol": "UBXN2B",
  "gene": "UniProtKB:Q14CS0",
  "term_label": "proteasome-mediated ubiquitin-dependent protein catabolic process",
  "term_id": "GO:0043161",
  "gene_name": "UBX domain-containing protein 2B"
}